{
  "gene_name": "Ubiquinol-cytochrome-c reductase complex assembly factor 5",
  "term_id": "UNKNOWN:0001",
  "gene_symbol": "UQCC5",
  "term_label": "Unknown molecular function",
  "gene": "UniProtKB:Q8WVI0"
}